histone H3Q5ser reader activity [GO:0140004] (molecular function) Relationships: is a type of histone H3 reader activity [GO:0140006] Definition: A histone reader that recognizes a histone H3 serotonylated at glutamine 5. Also known as: H3Q5-serotonin histone reader activity, H3Q5-serotonin modified histone binding References: PMID:34144982 Note: Comment: Note that the residue position corresponds to the canonical human H3 histone (UniProtKB:P84243); this residue is conserved across all eukaryotes. Residue 1 is the first residue following removal of the initiating Methionine (Met). Note that each histone is encoded by multiple genes, and sequences may vary across different genes within an organism.